ethanol binding [GO:0035276] (molecular function) Relationships: is_a GO:0043168; is a type of alcohol binding [GO:0043178] Definition: Binding to ethanol, CH(3)-CH(2)-OH. Sources: ISBN:0198506732